{
  "gene": "UniProtKB:Q96FK6",
  "term_label": "Unknown molecular function",
  "term_id": "UNKNOWN:0001",
  "gene_name": "WD repeat-containing protein 89",
  "gene_symbol": "WDR89"
}